{
  "gene_symbol": "BRWD1",
  "term_id": "UNKNOWN:0001",
  "term_label": "Unknown molecular function",
  "gene": "UniProtKB:Q9NSI6",
  "gene_name": "Bromodomain and WD repeat-containing protein 1"
}